{
  "gene": "UniProtKB:Q96LP6",
  "term_id": "UNKNOWN:0001",
  "term_label": "Unknown molecular function",
  "gene_name": "Uncharacterized protein C12orf42",
  "gene_symbol": "C12orf42"
}